{
  "gene_name": "Syntenin-2",
  "gene": "UniProtKB:Q9H190",
  "gene_symbol": "SDCBP2",
  "term_id": "GO:0005737",
  "term_label": "cytoplasm"
}